plant-type hypersensitive response [GO:0009626] (biological process) Relationships: is a type of cellular response to stress [GO:0033554]; is a type of symbiont-induced defense-related programmed cell death [GO:0034050]; is a type of innate immune response [GO:0045087] Regulation: regulated by regulation of plant-type hypersensitive response [GO:0010363]; negatively regulated by negative regulation of plant-type hypersensitive response [GO:0034051]; positively regulated by positive regulation of plant-type hypersensitive response [GO:0034052] Note: Note that term is to be used to annotate gene products in the plant. To annotate symbiont gene products that induce the hypersensitive response, consider using 'effector-mediated activation of plant hypersensitive response by symbiont' ; GO:0080185. Sources: ISBN:0582227089 Definition: The rapid, localized death of plant cells in response to invasion by a pathogen. Also known as: HR, HR-PCD, plant hypersensitive response